CMG complex assembly [GO:0140529] (biological process) Relationships: is a type of GO:0071163; is part of nuclear cell cycle DNA replication initiation [GO:1902315] Definition: The aggregation, arrangement and bonding together of a set of components to form the CMG complex, a protein complex that contains the GINS complex, Cdc45p, and the heterohexameric MCM complex, and that is involved in unwinding DNA during replication. The process begins when additional proteins (e.g. Cdc45 and Sld3) join the loaded, inactive double MCM hexamer at replication origins, and ends when Mcm10 triggers the separation of the Mcm2-7 double hexamers, forming two active CMG complexes. References: PMID:22718908, PMID:28501329